{
  "term_label": "calcium-dependent cell-cell adhesion",
  "gene_symbol": "CDH17",
  "gene": "UniProtKB:Q12864",
  "gene_name": "Cadherin-17",
  "term_id": "GO:0016339"
}